{
  "term_label": "peptide antigen assembly with MHC class II protein complex",
  "term_id": "GO:0002503",
  "gene_symbol": "HLA-DRB5",
  "gene": "UniProtKB:Q30154",
  "gene_name": "HLA class II histocompatibility antigen, DR beta 5 chain"
}